{
  "gene_symbol": "SEZ6L2",
  "term_id": "UNKNOWN:0001",
  "gene": "UniProtKB:Q6UXD5",
  "gene_name": "Seizure 6-like protein 2",
  "term_label": "Unknown molecular function"
}